{
  "gene_name": "tRNA methyltransferase 10 homolog C",
  "term_id": "GO:0005654",
  "gene": "UniProtKB:Q7L0Y3",
  "term_label": "nucleoplasm",
  "gene_symbol": "TRMT10C"
}